{
  "gene": "UniProtKB:Q9P1A6",
  "gene_symbol": "DLGAP2",
  "term_id": "GO:0098978",
  "term_label": "glutamatergic synapse",
  "gene_name": "Disks large-associated protein 2"
}